{
  "gene_symbol": "ENTPD8",
  "term_label": "plasma membrane",
  "gene_name": "Ectonucleoside triphosphate diphosphohydrolase 8",
  "term_id": "GO:0005886",
  "gene": "UniProtKB:Q5MY95"
}